{
  "gene_name": "Acid-sensing ion channel 4",
  "gene_symbol": "ASIC4",
  "term_label": "sodium ion transmembrane transport",
  "term_id": "GO:0035725",
  "gene": "UniProtKB:Q96FT7"
}